{
  "term_id": "GO:0000290",
  "gene_name": "U6 snRNA-associated Sm-like protein LSm1",
  "gene": "UniProtKB:O15116",
  "gene_symbol": "LSM1",
  "term_label": "deadenylation-dependent decapping of nuclear-transcribed mRNA"
}